{
  "term_id": "GO:0032133",
  "gene_symbol": "BIRC5",
  "gene_name": "Baculoviral IAP repeat-containing protein 5",
  "gene": "UniProtKB:O15392",
  "term_label": "chromosome passenger complex"
}